{
  "term_id": "GO:0070699",
  "term_label": "type II activin receptor binding",
  "gene": "UniProtKB:Q86UL8",
  "gene_name": "Membrane-associated guanylate kinase, WW and PDZ domain-containing protein 2",
  "gene_symbol": "MAGI2"
}